adhesion of symbiont to host endothelial cell [GO:0044652] (biological process) References: PMID:10066176 Sources: GOC:jl Definition: The attachment of a symbiont to a host endothelial cell via adhesion molecules, general stickiness etc., either directly or indirectly. Relationships: is_a adhesion of symbiont to host cell [GO:0044650]